{
  "term_id": "GO:0007420",
  "gene_name": "Nipped-B-like protein",
  "gene_symbol": "NIPBL",
  "gene": "UniProtKB:Q6KC79",
  "term_label": "brain development"
}